macrophage colony-stimulating factor production [GO:0036301] (BP) Regulation: regulated by regulation of macrophage colony-stimulating factor production [GO:1901256]; negatively regulated by negative regulation of macrophage colony-stimulating factor production [GO:1901257]; positively regulated by positive regulation of macrophage colony-stimulating factor production [GO:1901258] Sources: GOC:BHF, GOC:vk Definition: The appearance of macrophage colony-stimulating factor due to biosynthesis or secretion following a cellular stimulus, resulting in an increase in its intracellular or extracellular levels. Also known as: M-CSF production Relationships: is a type of cytokine production [GO:0001816]